interleukin-28 receptor complex [GO:0032002] (cellular component) Definition: A protein complex that binds interleukin-28 and interleukin-29. It is composed of an alpha and a beta receptor subunit (in human IFNLR1/IL28Ralpha & IL10RB) and either Interleukin-28 (IFNL2 or IFNL3) or Interleukin-29 (IFNL1). Relationships: is a type of plasma membrane signaling receptor complex [GO:0098802] Sources: GOC:rph Also known as: IL-28 receptor complex